{
  "term_label": "vesicle-mediated transport",
  "gene_name": "Cytohesin-1",
  "gene": "UniProtKB:Q15438",
  "gene_symbol": "CYTH1",
  "term_id": "GO:0016192"
}